regulation of transcription, start site selection [GO:0010630] (biological process) Sources: GOC:dph, GOC:tb Definition: Any process that modulates the frequency, rate or extent of the synthesis of either RNA on a template of DNA or DNA on a template of RNA by a mechanism that selects the start site along that template. Subtypes: GO:0001178 Relationships: is a type of regulation of nucleobase-containing compound metabolic process [GO:0019219]